endonucleolytic cleavage in ITS1 upstream of 5.8S rRNA from tricistronic rRNA transcript (SSU-rRNA, 5.8S rRNA, LSU-rRNA) [GO:0000464] (biological process) Definition: Endonucleolytic cleavage within Internal Transcribed Spacer 1 (ITS1) upstream of the 5.8S rRNA derived from an originally tricistronic rRNA transcript that contained the Small Subunit (SSU) rRNA, the 5.8S rRNA, and the Large Subunit (LSU) rRNA in that order from 5' to 3' along the primary transcript. In S. cerevisiae, this endonucleolytic cleavage within ITS1 initiates the maturation of the LSU and the 5.8S rRNAs. References: PMID:10690410 Sources: GOC:krc Also known as: endonucleolytic cleavage at A3 Relationships: is a type of endonucleolytic cleavage of tricistronic rRNA transcript (SSU-rRNA, 5.8S rRNA, LSU-rRNA) [GO:0000479]; is part of maturation of LSU-rRNA from tricistronic rRNA transcript (SSU-rRNA, 5.8S rRNA, LSU-rRNA) [GO:0000463]; is part of GO:0000466